{
  "term_label": "extracellular matrix organization",
  "term_id": "GO:0030198",
  "gene_symbol": "COL9A3",
  "gene": "UniProtKB:Q14050",
  "gene_name": "Collagen alpha-3(IX) chain"
}